{
  "gene": "UniProtKB:Q8TCG2",
  "gene_symbol": "PI4K2B",
  "gene_name": "Phosphatidylinositol 4-kinase type 2-beta",
  "term_label": "phosphatidylinositol phosphate biosynthetic process",
  "term_id": "GO:0046854"
}